{
  "term_label": "sulfate transmembrane transport",
  "gene": "UniProtKB:Q96RN1",
  "term_id": "GO:1902358",
  "gene_name": "Testis anion transporter 1",
  "gene_symbol": "SLC26A8"
}